{
  "gene_symbol": "LRP3",
  "gene": "UniProtKB:O75074",
  "term_id": "UNKNOWN:0002",
  "gene_name": "Low-density lipoprotein receptor-related protein 3",
  "term_label": "Unknown biological process"
}